{
  "term_id": "GO:0016559",
  "term_label": "peroxisome fission",
  "gene": "UniProtKB:O96011",
  "gene_symbol": "PEX11B",
  "gene_name": "Peroxisomal membrane protein 11B"
}